{
  "term_label": "Unknown cellular component",
  "gene_name": "Dynein axonemal assembly factor 3",
  "term_id": "UNKNOWN:0003",
  "gene": "UniProtKB:Q8N9W5",
  "gene_symbol": "DNAAF3"
}